erythritol kinase activity [GO:0047878] (MF) Definition: Catalysis of the reaction: ATP + erythritol = D-erythritol 4-phosphate + ADP + 2 H+. Sources: EC:2.7.1.27, RHEA:20708 Relationships: is a type of kinase activity [GO:0016301]; is a type of phosphotransferase activity, alcohol group as acceptor [GO:0016773] Also known as: ATP:erythritol 4-phosphotransferase activity, erythritol kinase (phosphorylating)